{
  "term_id": "GO:0005634",
  "gene": "UniProtKB:Q8NA58",
  "gene_symbol": "PNLDC1",
  "term_label": "nucleus",
  "gene_name": "Poly(A)-specific ribonuclease PNLDC1"
}